{
  "term_label": "retrograde vesicle-mediated transport, Golgi to endoplasmic reticulum",
  "gene_name": "Endoplasmic reticulum-Golgi intermediate compartment protein 2",
  "term_id": "GO:0006890",
  "gene_symbol": "ERGIC2",
  "gene": "UniProtKB:Q96RQ1"
}